positive regulation of collagen biosynthetic process [GO:0032967] (biological process) Sources: GOC:mah Definition: Any process that activates or increases the frequency, rate or extent of the chemical reactions and pathways resulting in the formation of collagen, any of a group of fibrous proteins of very high tensile strength that form the main component of connective tissue in animals. Also known as: positive regulation of collagen anabolism, positive regulation of collagen biosynthesis, positive regulation of collagen formation, positive regulation of collagen synthesis Relationships: is a type of positive regulation of biosynthetic process [GO:0009891]; is a type of positive regulation of collagen metabolic process [GO:0010714]; is a type of GO:0032965; RO_0002213 collagen biosynthetic process [GO:0032964]